pyrimidine-nucleoside phosphorylase activity [GO:0016154] (molecular function) Also known as: Py-NPase activity, pyrimidine-nucleoside:phosphate alpha-D-ribosyltransferase activity Sources: EC:2.4.2.2 Subtypes: uridine phosphorylase activity [GO:0004850], thymidine phosphorylase activity [GO:0009032], GO:0047847 Definition: Catalysis of the reaction: pyrimidine nucleoside + phosphate = pyrimidine + alpha-D-ribose 1-phosphate. Relationships: is_a GO:0016763